regulation of short-term synaptic potentiation [GO:1905512] (biological process) Definition: Any process that modulates the frequency, rate or extent of short-term synaptic potentiation. References: PMID:15470145 Sources: GOC:TermGenie, GOC:hjd, GO_REF:0000058 Also known as: regulation of synaptic facilitation Relationships: is a type of regulation of synaptic plasticity [GO:0048167]; regulates short-term synaptic potentiation [GO:1990926] Subtypes: negative regulation of short-term synaptic potentiation [GO:1905513], positive regulation of short-term synaptic potentiation [GO:1905514]